{
  "term_label": "natural killer cell mediated cytotoxicity",
  "gene": "UniProtKB:Q8TD07",
  "gene_symbol": "RAET1E",
  "gene_name": "Retinoic acid early transcript 1E",
  "term_id": "GO:0042267"
}